{
  "gene_symbol": "ABHD8",
  "term_id": "GO:0042171",
  "gene": "UniProtKB:Q96I13",
  "term_label": "lysophosphatidic acid acyltransferase activity",
  "gene_name": "Protein ABHD8"
}